{
  "term_id": "UNKNOWN:0001",
  "gene": "UniProtKB:Q7RTY7",
  "gene_symbol": "OVCH1",
  "term_label": "Unknown molecular function",
  "gene_name": "Ovochymase-1"
}